{
  "gene_name": "FAST kinase domain-containing protein 4",
  "term_label": "RNA binding",
  "gene_symbol": "TBRG4",
  "term_id": "GO:0003723",
  "gene": "UniProtKB:Q969Z0"
}